glycine dehydrogenase (cyanide-forming) activity [GO:0050622] (molecular function) Also known as: HCN synthase activity, glycine:acceptor oxidoreductase (hydrogen-cyanide-forming), hydrogen cyanide synthase activity Definition: Catalysis of the reaction: glycine + 2 A = HCN + CO2 + 2 AH2. Relationships: is a type of oxidoreductase activity, acting on the CH-NH2 group of donors [GO:0016638] Sources: RHEA:15821